{
  "term_label": "tRNA (guanine) methyltransferase activity",
  "gene_symbol": "THUMPD2",
  "gene_name": "THUMP domain-containing protein 2",
  "term_id": "GO:0016423",
  "gene": "UniProtKB:Q9BTF0"
}